{
  "gene_symbol": "GYS2",
  "term_label": "alpha-1,4-glucan glucosyltransferase (UDP-glucose donor) activity",
  "gene_name": "Glycogen [starch] synthase, liver",
  "gene": "UniProtKB:P54840",
  "term_id": "GO:0004373"
}